{
  "gene_name": "Fibroblast growth factor receptor substrate 2",
  "term_id": "GO:0005104",
  "term_label": "fibroblast growth factor receptor binding",
  "gene_symbol": "FRS2",
  "gene": "UniProtKB:Q8WU20"
}